{
  "gene_symbol": "SMARCD2",
  "gene_name": "SWI_SNF-related matrix-associated actin-dependent regulator of chromatin subfamily D member 2",
  "term_id": "GO:0005634",
  "term_label": "nucleus",
  "gene": "UniProtKB:Q92925"
}